phosphoenolpyruvate carboxykinase (GTP) activity [GO:0004613] (molecular function) Sources: EC:4.1.1.32 Definition: Catalysis of the reaction: GTP + oxaloacetate = GDP + phosphoenolpyruvate + CO2. Relationships: is a type of phosphoenolpyruvate carboxykinase activity [GO:0004611] Also known as: phosphoenolpyruvic carboxykinase, phosphoenolpyruvate carboxylase (GTP), GTP:oxaloacetate carboxy-lyase (adding GTP; phosphoenolpyruvate-forming), GTP:oxaloacetate carboxy-lyase (transphosphorylating), phosphoenolpyruvic carboxykinase (GTP), phosphoenolpyruvic carboxylase (GTP), phosphopyruvate (guanosine triphosphate) carboxykinase activity, phosphopyruvate carboxylase (GTP)